{
  "term_id": "GO:0140359",
  "gene_symbol": "ABCC6",
  "gene": "UniProtKB:O95255",
  "term_label": "ABC-type transporter activity",
  "gene_name": "ATP-binding cassette sub-family C member 6"
}